{
  "term_id": "GO:0045599",
  "term_label": "negative regulation of fat cell differentiation",
  "gene": "UniProtKB:P22413",
  "gene_symbol": "ENPP1",
  "gene_name": "Ectonucleotide pyrophosphatase_phosphodiesterase family member 1"
}